{
  "term_label": "Unknown biological process",
  "gene": "UniProtKB:Q8TB33",
  "gene_symbol": "LINC01560",
  "gene_name": "Putative uncharacterized protein encoded by LINC01560",
  "term_id": "UNKNOWN:0002"
}